sinapoyl spermidine:sinapoyl CoA N-acyltransferase activity [GO:0080089] (molecular function) Relationships: is a type of GO:0016410 References: PMID:19168716 Definition: Catalysis of the transfer of a sinapoyl group to a nitrogen atom on a sinapoyl spermidine molecule resulting in the formation of a disinapoyl spermidine derivative.